{
  "gene_symbol": "MFSD13A",
  "term_label": "Unknown cellular component",
  "gene": "UniProtKB:Q14CX5",
  "term_id": "UNKNOWN:0003",
  "gene_name": "Transmembrane protein 180"
}